{
  "gene_symbol": "TNFSF13B",
  "term_label": "lymphocyte homeostasis",
  "gene": "UniProtKB:Q9Y275",
  "gene_name": "Tumor necrosis factor ligand superfamily member 13B",
  "term_id": "GO:0002260"
}